{
  "gene": "UniProtKB:Q9NZV6",
  "gene_name": "Methionine-R-sulfoxide reductase B1",
  "gene_symbol": "MSRB1",
  "term_label": "peptide-methionine (R)-S-oxide reductase activity",
  "term_id": "GO:0033743"
}